{
  "term_id": "UNKNOWN:0003",
  "gene": "UniProtKB:P58418",
  "gene_name": "Clarin-1",
  "gene_symbol": "CLRN1",
  "term_label": "Unknown cellular component"
}